{
  "gene_name": "Carbonic anhydrase 2",
  "term_id": "GO:0004089",
  "term_label": "carbonate dehydratase activity",
  "gene": "UniProtKB:P00918",
  "gene_symbol": "CA2"
}